{
  "gene_symbol": "HS3ST3A1",
  "gene_name": "Heparan sulfate glucosamine 3-O-sulfotransferase 3A1",
  "term_id": "UNKNOWN:0003",
  "gene": "UniProtKB:Q9Y663",
  "term_label": "Unknown cellular component"
}